{
  "gene_name": "Receptor-type tyrosine-protein phosphatase gamma",
  "term_id": "GO:0031175",
  "gene": "UniProtKB:P23470",
  "gene_symbol": "PTPRG",
  "term_label": "neuron projection development"
}